carnitine shuttle [GO:0006853] (biological process) Note: See also the cellular component term 'mitochondrial inner membrane ; GO:0005743'. Relationships: is a type of long-chain fatty acid transport [GO:0015909]; is a type of intracellular lipid transport [GO:0032365]; is a type of fatty acid transmembrane transport [GO:1902001]; is a type of mitochondrial transmembrane transport [GO:1990542] Definition: The transfer of acyl groups to and from acyl-CoA molecules to form O-acylcarnitine, which can exchange across the mitochondrial inner membrane with unacylated carnitine. Sources: ISBN:0198547684